{
  "gene_symbol": "CD40LG",
  "term_id": "GO:0007166",
  "term_label": "cell surface receptor signaling pathway",
  "gene_name": "CD40 ligand",
  "gene": "UniProtKB:P29965"
}